{
  "gene_name": "Hormone-sensitive lipase",
  "term_id": "GO:0004806",
  "term_label": "triacylglycerol lipase activity",
  "gene_symbol": "LIPE",
  "gene": "UniProtKB:Q05469"
}